oral incubation [GO:0060747] (biological process) Relationships: is a type of GO:0060746 Sources: GOC:dph Definition: A parental behavior in which fertilized eggs are taken into the mouth and held until hatching.